{
  "gene_symbol": "ELOF1",
  "term_id": "GO:0008023",
  "gene_name": "Transcription elongation factor 1 homolog",
  "gene": "UniProtKB:P60002",
  "term_label": "transcription elongation factor complex"
}